{
  "gene_symbol": "HIGD1A",
  "term_id": "UNKNOWN:0001",
  "gene_name": "HIG1 domain family member 1A, mitochondrial",
  "gene": "UniProtKB:Q9Y241",
  "term_label": "Unknown molecular function"
}